{
  "term_id": "GO:0005634",
  "term_label": "nucleus",
  "gene": "UniProtKB:Q9UMX2",
  "gene_symbol": "OAZ3",
  "gene_name": "Ornithine decarboxylase antizyme 3"
}